{
  "gene_name": "Amyloid-beta A4 precursor protein-binding family A member 3",
  "gene": "UniProtKB:O96018",
  "term_id": "GO:0001540",
  "gene_symbol": "APBA3",
  "term_label": "amyloid-beta binding"
}